innate immune response activating cell surface receptor signaling pathway [GO:0002220] (biological process) Relationships: is a type of immune response-activating cell surface receptor signaling pathway [GO:0002429]; is a type of innate immune response-activating signaling pathway [GO:0002758] References: PMID:15199967 Sources: GOC:add, ISBN:0781735149 Definition: The series of molecular signals initiated by a ligand binding to a cell surface receptor that leads to the activation of an innate immune response. Subtypes: stimulatory killer cell immunoglobulin-like receptor signaling pathway [GO:0002222], stimulatory C-type lectin receptor signaling pathway [GO:0002223], cell surface pattern recognition receptor signaling pathway [GO:0002752] Also known as: activation of innate immune response by cell surface receptor signaling pathway, innate immune response activating cell surface receptor signalling pathway